adenosine 3',5'-bisphosphate transmembrane transporter activity [GO:0071077] (molecular function) Also known as: adenosine 3',5'-diphosphate transporter activity, adenosine 3'-phosphate-5'-phosphate transmembrane transporter activity Relationships: is_a adenine nucleotide transmembrane transporter activity [GO:0000295]; is a type of purine ribonucleotide transmembrane transporter activity [GO:0005346]; is part of adenosine 3',5'-bisphosphate transmembrane transport [GO:0071106] Definition: Enables the transfer of adenosine 3',5'-bisphosphate from one side of a membrane to the other. Sources: GOC:mah